{
  "gene_symbol": "MON1B",
  "gene": "UniProtKB:Q7L1V2",
  "gene_name": "Vacuolar fusion protein MON1 homolog B",
  "term_id": "GO:0035658",
  "term_label": "Mon1-Ccz1 complex"
}